{
  "gene": "UniProtKB:O14843",
  "term_id": "GO:0007186",
  "term_label": "G protein-coupled receptor signaling pathway",
  "gene_symbol": "FFAR3",
  "gene_name": "Free fatty acid receptor 3"
}